angiotensin type II receptor activity [GO:0004945] (molecular function) Relationships: is a type of GO:0001595 Definition: An angiotensin receptor activity that acts via Gi protein coupling and cGMP (NO) generation, and may also act via additional signaling mechanisms. References: PMID:10977869 Sources: GOC:mah